calcium-dependent protein binding [GO:0048306] (molecular function) Relationships: is a type of protein binding [GO:0005515]; BFO_0000051 GO:0005509 References: PMID:10485905 Sources: GOC:jid Definition: Binding to a protein or protein complex in the presence of calcium. Subtypes: calcium-dependent outer dynein arm binding [GO:0120152]